{
  "term_label": "prevention of polyspermy",
  "term_id": "GO:0060468",
  "gene_symbol": "ZP1",
  "gene_name": "Zona pellucida sperm-binding protein 1",
  "gene": "UniProtKB:P60852"
}